nucleobase-containing compound catabolic process [GO:0034655] (biological process) Relationships: is a type of nucleobase-containing compound metabolic process [GO:0006139]; is a type of catabolic process [GO:0009056] Also known as: nucleobase, nucleoside, nucleotide and nucleic acid breakdown, nucleobase, nucleoside, nucleotide and nucleic acid catabolism, nucleobase, nucleoside, nucleotide and nucleic acid degradation, nucleobase, nucleoside, nucleotide and nucleic acid catabolic process Subtypes: GO:0034656, nucleic acid catabolic process [GO:0141188], nucleoside phosphate catabolic process [GO:1901292] Sources: GOC:mah Definition: The chemical reactions and pathways resulting in the breakdown of nucleobases, nucleosides, nucleotides and nucleic acids.